{
  "gene_name": "Interferon-induced protein 44-like",
  "gene": "UniProtKB:Q53G44",
  "term_id": "UNKNOWN:0001",
  "term_label": "Unknown molecular function",
  "gene_symbol": "IFI44L"
}